{
  "gene": "UniProtKB:Q9P0M2",
  "gene_name": "A-kinase anchor protein 7 isoform gamma",
  "term_label": "cytosol",
  "gene_symbol": "AKAP7",
  "term_id": "GO:0005829"
}